{
  "term_id": "GO:0030317",
  "gene": "UniProtKB:Q6ZNM6",
  "gene_symbol": "SPMIP10",
  "gene_name": "Testis-expressed protein 43",
  "term_label": "flagellated sperm motility"
}